negative regulation of lipoprotein metabolic process [GO:0050748] (BP) Sources: GOC:ai Also known as: down regulation of lipoprotein metabolic process, down-regulation of lipoprotein metabolic process, downregulation of lipoprotein metabolic process, negative regulation of lipoprotein metabolism, inhibition of lipoprotein metabolic process Definition: Any process that stops, prevents, or reduces the frequency, rate or extent of the chemical reactions and pathways involving lipoproteins, any conjugated, water-soluble protein in which the nonprotein group consists of a lipid or lipids. Relationships: is a type of regulation of lipoprotein metabolic process [GO:0050746]; is a type of negative regulation of protein metabolic process [GO:0051248]; negatively regulates lipoprotein metabolic process [GO:0042157] Subtypes: negative regulation of lipoprotein oxidation [GO:0034443], negative regulation of protein lipidation [GO:1903060]